{
  "term_label": "mitochondrion",
  "gene_name": "Branched-chain-amino-acid aminotransferase, cytosolic",
  "gene_symbol": "BCAT1",
  "term_id": "GO:0005739",
  "gene": "UniProtKB:P54687"
}